{
  "gene_name": "Testis-expressed protein 11",
  "gene": "UniProtKB:Q8IYF3",
  "term_label": "central element",
  "term_id": "GO:0000801",
  "gene_symbol": "TEX11"
}